{
  "term_label": "stress fiber",
  "gene": "UniProtKB:Q99501",
  "gene_symbol": "GAS2L1",
  "gene_name": "GAS2-like protein 1",
  "term_id": "GO:0001725"
}